{
  "gene": "UniProtKB:P35462",
  "term_id": "GO:0051481",
  "gene_name": "D(3) dopamine receptor",
  "term_label": "negative regulation of cytosolic calcium ion concentration",
  "gene_symbol": "DRD3"
}